{
  "term_id": "GO:0009897",
  "gene_symbol": "ACKR4",
  "gene_name": "Atypical chemokine receptor 4",
  "term_label": "external side of plasma membrane",
  "gene": "UniProtKB:Q9NPB9"
}